{
  "gene": "UniProtKB:P01148",
  "term_label": "gonadotropin hormone-releasing hormone activity",
  "gene_symbol": "GNRH1",
  "gene_name": "Progonadoliberin-1",
  "term_id": "GO:0005183"
}